hypothalamus gonadotrophin-releasing hormone neuron development [GO:0021888] (biological process) Definition: The process whose specific outcome is the progression of a hypothalamus gonadotrophin-releasing hormone neuron over time, from initial commitment of its fate, to the fully functional differentiated cell. Also known as: hypothalamus gonadotropin-releasing hormone neuron development Relationships: is a type of GO:0021884; is part of hypothalamus gonadotrophin-releasing hormone neuron differentiation [GO:0021886] References: PMID:12626695 Sources: GOC:cls, GOC:dgh, GOC:dph, GOC:jid, GO_REF:0000021